{
  "gene": "UniProtKB:P49789",
  "gene_symbol": "FHIT",
  "gene_name": "Bis(5'-adenosyl)-triphosphatase",
  "term_id": "GO:0047710",
  "term_label": "bis(5'-adenosyl)-triphosphatase activity"
}